{
  "term_label": "regulation of transcription by RNA polymerase II",
  "gene_name": "Homeobox protein Hox-A1",
  "gene": "UniProtKB:P49639",
  "term_id": "GO:0006357",
  "gene_symbol": "HOXA1"
}